{
  "gene_symbol": "NTRK1",
  "term_id": "GO:0043121",
  "gene": "UniProtKB:P04629",
  "gene_name": "High affinity nerve growth factor receptor",
  "term_label": "neurotrophin binding"
}